intracellular transport of virus [GO:0075733] (biological process) Definition: The directed movement of a virus, or part of a virus, within the host cell. References: PMID:11733033 Sources: GOC:ai, GOC:bf, GOC:jl Also known as: egress of virus within host cell, intracellular transport of viral material, movement of virus within host cell, viral genome transport in host cell, intracellular virion transport, viral egress Relationships: is a type of biological process involved in symbiotic interaction [GO:0044403]; is a type of transport of virus [GO:0046794]; is part of GO:0019058; occurs in host cell [GO:0043657] Subtypes: microtubule-dependent intracellular transport of viral material [GO:0075519], GO:0075520, GO:0075606, viral penetration into host nucleus [GO:0075732] Regulation: regulated by GO:1901252; negatively regulated by negative regulation of intracellular transport of viral material [GO:1901253]; positively regulated by positive regulation of intracellular transport of viral material [GO:1901254]